{
  "gene_name": "Sodium-dependent phosphate transport protein 4",
  "gene_symbol": "SLC17A3",
  "gene": "UniProtKB:O00476",
  "term_id": "GO:0042910",
  "term_label": "xenobiotic transmembrane transporter activity"
}